{
  "gene_symbol": "SMAD5",
  "gene_name": "Mothers against decapentaplegic homolog 5",
  "term_label": "regulation of transcription by RNA polymerase II",
  "term_id": "GO:0006357",
  "gene": "UniProtKB:Q99717"
}